{
  "gene_symbol": "NR1H4",
  "term_label": "bile acid binding",
  "term_id": "GO:0032052",
  "gene_name": "Bile acid receptor",
  "gene": "UniProtKB:Q96RI1"
}